{
  "gene": "UniProtKB:Q9H0B8",
  "term_label": "glycosaminoglycan binding",
  "term_id": "GO:0005539",
  "gene_name": "Cysteine-rich secretory protein LCCL domain-containing 2",
  "gene_symbol": "CRISPLD2"
}